negative regulation of lipoprotein particle clearance [GO:0010985] (biological process) Subtypes: negative regulation of very-low-density lipoprotein particle clearance [GO:0010916], negative regulation of high-density lipoprotein particle clearance [GO:0010987], negative regulation of low-density lipoprotein particle clearance [GO:0010989] Definition: Any process that decreases the rate, frequency, or extent of lipoprotein particle clearance. Lipoprotein particle clearance is the process in which a lipoprotein particle is removed from the blood via receptor-mediated endocytosis and its constituent parts degraded. Sources: GOC:BHF, GOC:dph, GOC:tb Relationships: is a type of regulation of lipoprotein particle clearance [GO:0010984]; is a type of negative regulation of multicellular organismal process [GO:0051241]; negatively regulates plasma lipoprotein particle clearance [GO:0034381]